spherical high-density lipoprotein particle [GO:0034366] (cellular component) Also known as: mature HDL, mature high-density lipoprotein particle, spherical HDL Sources: GOC:BHF, GOC:expert_pt, GOC:mah, GOC:rl Relationships: is a type of high-density lipoprotein particle [GO:0034364] Definition: A mature high-density lipoprotein (HDL) particle, converted from discoidal HDL particles following the esterification of cholesterol in the particle by phosphatidylcholine-sterol O-acyltransferase (lecithin cholesterol acyltransferase; LCAT).